{
  "gene_name": "Histone-lysine N-methyltransferase SUV39H1",
  "gene": "UniProtKB:O43463",
  "term_label": "nucleus",
  "term_id": "GO:0005634",
  "gene_symbol": "SUV39H1"
}